metanephric interstitial fibroblast development [GO:0072259] (biological process) Sources: GOC:mtg_kidney_jan10 Relationships: is a type of renal interstitial fibroblast development [GO:0072141]; is part of metanephric interstitial fibroblast differentiation [GO:0072258] Definition: The process whose specific outcome is the progression of a metanephric interstitial fibroblast over time, from its formation to the mature structure. Also known as: metanephros interstitial cell development